ammonium ion binding [GO:0070405] (molecular function) Also known as: ammonium binding Sources: CHEBI:28938, GOC:ecd Definition: Binding to ammonium ions (NH4+). Relationships: is a type of cation binding [GO:0043169]